{
  "term_label": "Unknown biological process",
  "term_id": "UNKNOWN:0002",
  "gene_name": "Testis-expressed protein 10",
  "gene": "UniProtKB:Q9NXF1",
  "gene_symbol": "TEX10"
}